{
  "gene": "UniProtKB:Q14C86",
  "term_id": "UNKNOWN:0002",
  "gene_name": "GTPase-activating protein and VPS9 domain-containing protein 1",
  "gene_symbol": "GAPVD1",
  "term_label": "Unknown biological process"
}